penile erection [GO:0043084] (biological process) Relationships: is a type of multicellular organismal reproductive process [GO:0048609]; BFO_0000050 copulation [GO:0007620] Regulation: regulated by regulation of penile erection [GO:0060405]; RO_0002213 by positive regulation of penile erection [GO:0060406]; RO_0002212 by negative regulation of penile erection [GO:0060407] Sources: GOC:jl, Wikipedia:Penile_erection Definition: The hardening, enlarging and rising of the penis which often occurs in the sexually aroused male and enables sexual intercourse. Achieved by increased inflow of blood into the vessels of erectile tissue, and decreased outflow.